{
  "gene_symbol": "RPL22L1",
  "gene_name": "Ribosomal protein eL22-like",
  "gene": "UniProtKB:Q6P5R6",
  "term_label": "structural constituent of ribosome",
  "term_id": "GO:0003735"
}